{
  "gene_symbol": "FGF1",
  "gene_name": "Fibroblast growth factor 1",
  "gene": "UniProtKB:P05230",
  "term_label": "positive regulation of cell population proliferation",
  "term_id": "GO:0008284"
}